AMP dimethylallyltransferase activity [GO:0009824] (molecular function) Relationships: is a type of transferase activity, transferring alkyl or aryl (other than methyl) groups [GO:0016765] Sources: RHEA:15285 Definition: Catalysis of the reaction: AMP + dimethylallyl diphosphate = N(6)-(dimethylallyl)adenosine 5'-phosphate + diphosphate. Also known as: adenylate isopentenyltransferase activity, cytokinin synthase activity, isopentenyltransferase activity, 2-isopentenyl-diphosphate:AMP 2-isopentenyltransferase activity, 2-isopentenyl-diphosphate:AMP delta2-isopentenyltransferase activity, adenylate dimethylallyltransferase (AMP-dependent) activity, adenylate dimethylallyltransferase activity, dimethylallyl-diphosphate:AMP dimethylallyltransferase activity